{
  "term_id": "GO:0005764",
  "gene_name": "Rab-interacting lysosomal protein",
  "term_label": "lysosome",
  "gene_symbol": "RILP",
  "gene": "UniProtKB:Q96NA2"
}